{
  "gene_name": "Low affinity immunoglobulin gamma Fc region receptor II-b",
  "gene_symbol": "FCGR2B",
  "term_id": "GO:0007166",
  "gene": "UniProtKB:P31994",
  "term_label": "cell surface receptor signaling pathway"
}